{
  "gene_symbol": "PHEX",
  "term_id": "GO:0005886",
  "term_label": "plasma membrane",
  "gene_name": "Phosphate-regulating neutral endopeptidase PHEX",
  "gene": "UniProtKB:P78562"
}